{
  "term_id": "GO:0005516",
  "gene_symbol": "CAMKV",
  "term_label": "calmodulin binding",
  "gene": "UniProtKB:Q8NCB2",
  "gene_name": "CaM kinase-like vesicle-associated protein"
}